establishment of mitotic spindle orientation involved in growth plate cartilage chondrocyte division [GO:0003425] (biological process) Sources: GOC:ascb_2009, GOC:dph, GOC:tb Definition: A cell cycle process that sets the alignment of mitotic spindle relative to other cellular structures and contributes to oriented chondrocyte division in the growth plate. Relationships: is a type of establishment of mitotic spindle orientation [GO:0000132]; is a type of GO:0003426; is a type of microtubule cytoskeleton organization involved in establishment of planar polarity [GO:0090176]